{
  "term_id": "GO:0071949",
  "gene_name": "Hydroxyproline dehydrogenase",
  "gene": "UniProtKB:Q9UF12",
  "gene_symbol": "PRODH2",
  "term_label": "FAD binding"
}